{
  "term_id": "GO:0046856",
  "gene_name": "Phosphatidylinositol 3,4,5-trisphosphate 3-phosphatase and dual-specificity protein phosphatase PTEN",
  "term_label": "phosphatidylinositol dephosphorylation",
  "gene": "UniProtKB:P60484",
  "gene_symbol": "PTEN"
}